{
  "term_label": "DNA damage response",
  "gene_name": "SMC5-SMC6 complex localization factor protein 2",
  "gene_symbol": "SLF2",
  "gene": "UniProtKB:Q8IX21",
  "term_id": "GO:0006974"
}